{
  "gene": "UniProtKB:Q96BD5",
  "gene_symbol": "PHF21A",
  "term_label": "Unknown biological process",
  "gene_name": "PHD finger protein 21A",
  "term_id": "UNKNOWN:0002"
}